{
  "term_label": "Unknown biological process",
  "gene_symbol": "PCOLCE2",
  "term_id": "UNKNOWN:0002",
  "gene_name": "Procollagen C-endopeptidase enhancer 2",
  "gene": "UniProtKB:Q9UKZ9"
}